{
  "gene_name": "Acetyl-CoA carboxylase 2",
  "term_id": "GO:0005739",
  "gene_symbol": "ACACB",
  "term_label": "mitochondrion",
  "gene": "UniProtKB:O00763"
}